S-adenosylhomocysteine deaminase activity [GO:0050270] (molecular function) Relationships: is a type of hydrolase activity, acting on carbon-nitrogen (but not peptide) bonds, in cyclic amidines [GO:0016814]; is a type of GO:0019239 Definition: Catalysis of the reaction: S-adenosyl-L-homocysteine + H2O + H+ = S-inosyl-L-homocysteine + NH4. Sources: EC:3.5.4.28, RHEA:20716 Also known as: S-adenosyl-L-homocysteine aminohydrolase activity, adenosylhomocysteine deaminase activity